(+)-larreatricin metabolic process [GO:1901709] (biological process) Relationships: is a type of lignan metabolic process [GO:0009806]; is a type of GO:0018958 Also known as: (+)-larreatricin metabolism Definition: The chemical reactions and pathways involving (+)-larreatricin. References: PMID:12960376 Sources: GOC:TermGenie